{
  "gene_name": "E3 ubiquitin-protein ligase XIAP",
  "gene_symbol": "XIAP",
  "term_id": "GO:0031398",
  "term_label": "positive regulation of protein ubiquitination",
  "gene": "UniProtKB:P98170"
}